{
  "term_id": "GO:0005737",
  "gene_name": "Tubulin beta-4B chain",
  "term_label": "cytoplasm",
  "gene_symbol": "TUBB4B",
  "gene": "UniProtKB:P68371"
}